{
  "term_id": "UNKNOWN:0003",
  "gene_symbol": "TMEM158",
  "term_label": "Unknown cellular component",
  "gene_name": "Transmembrane protein 158",
  "gene": "UniProtKB:Q8WZ71"
}